{
  "gene": "UniProtKB:Q6NT32",
  "gene_symbol": "CES5A",
  "term_id": "UNKNOWN:0003",
  "term_label": "Unknown cellular component",
  "gene_name": "Carboxylesterase 5A"
}